oxidoreductase activity, acting on X-H and Y-H to form an X-Y bond [GO:0046992] (molecular function) Subtypes: thyroxine 5'-deiodinase activity [GO:0004800], 2,4-dichlorobenzoyl-CoA reductase activity [GO:0018516], GO:0018698, GO:0033798, oxidoreductase activity, acting on X-H and Y-H to form an X-Y bond, with oxygen as acceptor [GO:0046993], beta-cyclopiazonate dehydrogenase activity [GO:0050448], oxidoreductase activity, acting on X-H and Y-H to form an X-Y bond, with a disulfide as acceptor [GO:0050485], tetrachloroethene reductive dehalogenase activity [GO:0050629], trichloroethene reductive dehalogenase activity [GO:0050697], trichloro-p-hydroquinone reductive dehalogenase activity [GO:0052690], iodotyrosine deiodinase activity [GO:0140616] Also known as: oxidoreductase activity, acting on X-H and Y-H to form an X-Y bond, with other acceptors Relationships: is a type of oxidoreductase activity [GO:0016491] Sources: GOC:ai Definition: Catalysis of an oxidation-reduction (redox) reaction in which X-H and Y-H form X-Y.